{
  "gene": "UniProtKB:A8MXK1",
  "gene_symbol": "VSTM5",
  "term_id": "GO:0006955",
  "term_label": "immune response",
  "gene_name": "V-set and transmembrane domain-containing protein 5"
}